{
  "term_id": "UNKNOWN:0001",
  "gene_symbol": "FAM90A24P",
  "gene_name": "Putative protein FAM90A24P",
  "gene": "UniProtKB:P0C7X0",
  "term_label": "Unknown molecular function"
}